{
  "term_id": "GO:0035987",
  "gene": "UniProtKB:Q99715",
  "gene_symbol": "COL12A1",
  "gene_name": "Collagen alpha-1(XII) chain",
  "term_label": "endodermal cell differentiation"
}